{
  "gene": "UniProtKB:A1A5D9",
  "gene_symbol": "BICDL2",
  "term_id": "UNKNOWN:0003",
  "gene_name": "BICD family-like cargo adapter 2",
  "term_label": "Unknown cellular component"
}